{
  "term_id": "GO:0000981",
  "gene_symbol": "ZNF519",
  "gene": "UniProtKB:Q8TB69",
  "term_label": "DNA-binding transcription factor activity, RNA polymerase II-specific",
  "gene_name": "Zinc finger protein 519"
}